cysteine catabolic process [GO:0009093] (biological process) Definition: The chemical reactions and pathways resulting in the breakdown of cysteine, 2-amino-3-mercaptopropanoic acid. Sources: GOC:go_curators Also known as: cysteine breakdown, cysteine catabolism, cysteine degradation Relationships: is a type of sulfur amino acid catabolic process [GO:0000098]; is a type of cysteine metabolic process [GO:0006534]; is a type of GO:1901606 Subtypes: GO:0019447, L-cysteine catabolic process [GO:0019448]